regulation of proteolysis involved in protein catabolic process [GO:1903050] (biological process) Also known as: regulation of peptidolysis involved in cellular protein catabolic process, regulation of peptidolysis involved in cellular protein catabolism, regulation of proteolysis involved in cellular protein catabolic process, regulation of peptidolysis during cellular protein catabolic process, regulation of peptidolysis during cellular protein catabolism, regulation of proteolysis during cellular protein catabolic process, regulation of proteolysis during cellular protein catabolism Note: overexpression of cathepsin C propeptide significantly increased the degradation of intestinal alkaline phosphatase (IAP) Definition: Any process that modulates the frequency, rate or extent of proteolysis involved in cellular catabolic process. References: PMID:18307834 Sources: GOC:BHF, GOC:TermGenie, GOC:rl, GO_REF:0000058 Subtypes: regulation of proteolysis associated with antigen processing and presentation [GO:0002628], GO:0061136, GO:1903051, positive regulation of proteolysis involved in protein catabolic process [GO:1903052], regulation of ubiquitin-dependent protein catabolic process [GO:2000058] Relationships: is a type of regulation of proteolysis [GO:0030162]; regulates proteolysis involved in protein catabolic process [GO:0051603]